{
  "term_label": "DNA-binding transcription factor activity, RNA polymerase II-specific",
  "gene": "UniProtKB:Q13029",
  "gene_symbol": "PRDM2",
  "term_id": "GO:0000981",
  "gene_name": "PR domain zinc finger protein 2"
}